{
  "gene_name": "Gigaxonin",
  "gene_symbol": "GAN",
  "gene": "UniProtKB:Q9H2C0",
  "term_id": "GO:1990756",
  "term_label": "ubiquitin-like ligase-substrate adaptor activity"
}